rifamycin-B oxidase activity [GO:0050264] (molecular function) Also known as: rifamycin-B-oxidase activity, rifamycin B oxidase activity, rifamycin-B:oxygen oxidoreductase activity Definition: Catalysis of the reaction: 2 H+ + O2 + rifamycin B = H2O2 + rifamycin O. Sources: EC:1.10.3.6, RHEA:11292 Relationships: is a type of GO:0016682